{
  "gene": "UniProtKB:Q8NGG4",
  "term_id": "GO:0004984",
  "term_label": "olfactory receptor activity",
  "gene_name": "Olfactory receptor 8H1",
  "gene_symbol": "OR8H1"
}